endocrine pancreas development [GO:0031018] (BP) Sources: GOC:cvs Definition: The process whose specific outcome is the progression of the endocrine pancreas over time, from its formation to the mature structure. The endocrine pancreas is made up of islet cells that produce insulin, glucagon and somatostatin. Relationships: is_a anatomical structure development [GO:0048856]; BFO_0000050 pancreas development [GO:0031016]; is part of endocrine system development [GO:0035270]